ventricular cardiac myofibril assembly [GO:0055005] (biological process) Sources: GOC:devbiol Also known as: ventricular heart myofibril development, ventricular cardiac myofibril development Relationships: is a type of cardiac myofibril assembly [GO:0055003]; is part of ventricular cardiac muscle cell development [GO:0055015] Definition: The process whose specific outcome is the progression of the ventricular cardiac myofibril over time, from its formation to the mature structure. A cardiac myofibril is a myofibril specific to cardiac muscle cells.